{
  "gene_name": "Brain-specific angiogenesis inhibitor 1-associated protein 2-like protein 2",
  "gene_symbol": "BAIAP2L2",
  "term_label": "nucleoplasm",
  "term_id": "GO:0005654",
  "gene": "UniProtKB:Q6UXY1"
}